{
  "term_label": "canonical Wnt signaling pathway",
  "term_id": "GO:0060070",
  "gene": "UniProtKB:P14923",
  "gene_symbol": "JUP",
  "gene_name": "Junction plakoglobin"
}